{
  "gene_name": "Testis-expressed protein 19",
  "term_label": "placenta development",
  "gene_symbol": "TEX19",
  "gene": "UniProtKB:Q8NA77",
  "term_id": "GO:0001890"
}